{
  "gene_symbol": "CHRND",
  "term_id": "GO:0005886",
  "gene_name": "Acetylcholine receptor subunit delta",
  "gene": "UniProtKB:Q07001",
  "term_label": "plasma membrane"
}